{
  "gene_symbol": "IFTAP",
  "gene": "UniProtKB:Q86VG3",
  "term_id": "GO:0007340",
  "gene_name": "Intraflagellar transport-associated protein",
  "term_label": "acrosome reaction"
}